{
  "gene_symbol": "STAG3L2",
  "gene": "UniProtKB:P0CL84",
  "term_label": "Unknown cellular component",
  "term_id": "UNKNOWN:0003",
  "gene_name": "Putative STAG3-like protein 2"
}